{
  "term_label": "neuron development",
  "gene_symbol": "ALX3",
  "gene_name": "Homeobox protein aristaless-like 3",
  "term_id": "GO:0048666",
  "gene": "UniProtKB:O95076"
}